quercetin 7-O-methyltransferase activity [GO:0102432] (molecular function) Sources: RHEA:73115 Relationships: is a type of methyltransferase activity [GO:0008168] Definition: Catalysis of the reaction: quercetin + S-adenosyl-L-methionine = H+ + rhamnetin + S-adenosyl-L-homocysteine.